{
  "gene": "UniProtKB:Q8TB22",
  "gene_symbol": "SPATA20",
  "term_id": "UNKNOWN:0003",
  "gene_name": "Spermatogenesis-associated protein 20",
  "term_label": "Unknown cellular component"
}